anaerobic 2-aminobenzoate metabolic process [GO:0018870] (biological process) Sources: GOC:ai Definition: The chemical reactions and pathways resulting in the breakdown of 2-aminobenzoate, a derivative of benzoic acid with an NH2 group attached to C2, that occurs in the absence of oxygen. Relationships: is a type of anthranilate metabolic process [GO:0043420] Also known as: anaerobic 2-aminobenzoate metabolism